{
  "gene_name": "Unconventional myosin-Ie",
  "gene_symbol": "MYO1E",
  "term_id": "GO:0006897",
  "gene": "UniProtKB:Q12965",
  "term_label": "endocytosis"
}